{
  "gene": "UniProtKB:Q52LG2",
  "term_label": "Unknown molecular function",
  "gene_symbol": "KRTAP13-2",
  "gene_name": "Keratin-associated protein 13-2",
  "term_id": "UNKNOWN:0001"
}